{
  "gene_name": "tRNA N6-adenosine threonylcarbamoyltransferase, mitochondrial",
  "gene_symbol": "OSGEPL1",
  "gene": "UniProtKB:Q9H4B0",
  "term_id": "UNKNOWN:0002",
  "term_label": "Unknown biological process"
}